histone H3K27me2/H3K27me3 demethylase activity [GO:0071558] (molecular function) Note: Comment: Note that the residue position corresponds to the canonical human H3 histone (UniProtKB:P84243); this residue is conserved across all eukaryotes. Residue 1 is the first residue following removal of the initiating Methionine (Met). Note that each histone is encoded by multiple genes, and sequences may vary across different genes within an organism. Definition: Catalysis of the removal of a methyl group from a tri- or a dimethyl-lysine residue at position 27 of the histone H3 protein. This is a dioxygenase reaction that is dependent on Fe(II) and 2-oxoglutarate. References: PMID:20622853 Sources: GOC:sp Also known as: histone demethylase activity (H3-K27 specific), histone H3-tri/di-methyl-lysine-27 demethylase activity, histone H3K27me2 demethylase activity, histone H3K27me3 demethylase activity Relationships: is a type of 2-oxoglutarate-dependent dioxygenase activity [GO:0016706]; is_a histone H3 demethylase activity [GO:0141052]